pH-gated monoatomic ion channel activity [GO:0160128] (molecular function) Definition: Enables the transmembrane transfer of an inorganic ion by a channel that opens in response to a change in proton concentration (pH). Subtypes: pH-gated chloride channel activity [GO:0061797], GO:0160125, pH-gated calcium channel activity [GO:0160126] Also known as: proton-gated ion channel activity, acid-sensing ion channel activity References: PMID:17167423, PMID:29513651 Relationships: is_a ligand-gated monoatomic ion channel activity [GO:0015276] Note: While the term suggest this activity may be proton-gated, the mechanism of pH-gating for transporters is by protonation of specific residues in the protein, and not by H+ binding.